{
  "gene_name": "Transcription factor Jun",
  "gene": "UniProtKB:P05412",
  "term_label": "positive regulation of transcription by RNA polymerase II",
  "gene_symbol": "JUN",
  "term_id": "GO:0045944"
}